{
  "gene_name": "LIM domain-containing protein ajuba",
  "term_id": "GO:0005667",
  "gene_symbol": "AJUBA",
  "gene": "UniProtKB:Q96IF1",
  "term_label": "transcription regulator complex"
}